{
  "gene_symbol": "LRRIQ4",
  "term_label": "Unknown biological process",
  "gene": "UniProtKB:A6NIV6",
  "gene_name": "Leucine-rich repeat and IQ domain-containing protein 4",
  "term_id": "UNKNOWN:0002"
}